positive regulation of mitophagy [GO:1901526] (biological process) Definition: Any process that activates or increases the frequency, rate or extent of mitophagy. Also known as: positive regulation of macromitophagy, up regulation of macromitophagy, up-regulation of macromitophagy, upregulation of macromitophagy, activation of macromitophagy Subtypes: positive regulation of type 2 mitophagy [GO:1905091] Sources: GOC:TermGenie Relationships: is a type of positive regulation of macroautophagy [GO:0016239]; is a type of regulation of mitophagy [GO:1901524]; is a type of positive regulation of autophagy of mitochondrion [GO:1903599]; RO_0002213 mitophagy [GO:0000423]